{
  "gene_symbol": "RGS22",
  "term_label": "Unknown biological process",
  "gene_name": "Regulator of G-protein signaling 22",
  "gene": "UniProtKB:Q8NE09",
  "term_id": "UNKNOWN:0002"
}